host cell envelope [GO:0044230] (cellular component) Definition: An envelope that surrounds a bacterial host cell and includes the host cytoplasmic membrane and everything external, encompassing the host periplasmic space, host cell wall, and host outer membrane if present. Relationships: is a type of host cell part [GO:0033643] Sources: GOC:rph